ABC-type peptide antigen transporter activity [GO:0015433] (molecular function) Also known as: peptide antigen transporter activity, ATP-dependent peptide antigen transmembrane transporter activity, major histocompatibility peptide transporter activity, peptide antigen-transporting ATPase activity, peptide antigen ABC transporter, ATPase-coupled peptide antigen transmembrane transporter activity Relationships: is a type of ABC-type peptide transporter activity [GO:0015440] Definition: Catalysis of the reaction: peptide antigen(in) + ATP = peptide antigen(out) + ADP + phosphate. Sources: TC:3.A.1.209.1